{
  "term_label": "protein tag activity",
  "term_id": "GO:0031386",
  "gene_name": "Ubiquitin-ribosomal protein eS31 fusion protein",
  "gene": "UniProtKB:P62979",
  "gene_symbol": "RPS27A"
}